proclavaminate amidinohydrolase activity [GO:0033972] (molecular function) Definition: Catalysis of the reaction: amidinoproclavaminate + H2O = proclavaminate + urea. Sources: EC:3.5.3.22, RHEA:17001 Relationships: is a type of GO:0016813 Also known as: PAH, proclavaminate amidino hydrolase activity, proclavaminic acid amidino hydrolase activity